mitotic G2 cell cycle arrest in response to glucose starvation [GO:0036227] (biological process) References: PMID:958201 Sources: GOC:al, GOC:mah, GOC:mtg_cell_cycle Relationships: is_a regulation of cell cycle [GO:0051726] Definition: The process in which the mitotic cell cycle is halted during G2 phase as a result of deprivation of glucose.